fructokinase activity [GO:0008865] (molecular function) Relationships: is a type of GO:0004396 Also known as: ATP:D-fructose 6-phosphotransferase activity, D-fructokinase activity, D-fructose(D-mannose)kinase activity, fructokinase (phosphorylating) Definition: Catalysis of the reaction: ATP + D-fructose = ADP + D-fructose 6-phosphate. Sources: EC:2.7.1.4